chromoplast envelope [GO:0031898] (cellular component) Definition: The double lipid bilayer enclosing the chromoplast and separating its contents from the rest of the cytoplasm; includes the intermembrane space. Relationships: is a type of GO:0009526; BFO_0000050 chromoplast [GO:0009509] Sources: GOC:pz